{
  "term_id": "GO:0005783",
  "term_label": "endoplasmic reticulum",
  "gene_name": "Dol-P-Glc:Glc(2)Man(9)GlcNAc(2)-PP-Dol alpha-1,2-glucosyltransferase",
  "gene_symbol": "ALG10",
  "gene": "UniProtKB:Q5BKT4"
}